{
  "gene": "UniProtKB:Q9NRD8",
  "term_id": "GO:0006952",
  "gene_name": "Dual oxidase 2",
  "gene_symbol": "DUOX2",
  "term_label": "defense response"
}